positive regulation of cellular process [GO:0048522] (biological process) Subtypes: GO:0003353, positive regulation of cell population proliferation [GO:0008284], positive regulation of metabolic process [GO:0009893], positive regulation of cell communication [GO:0010647], positive regulation of lipid storage [GO:0010884], positive regulation of cell growth [GO:0030307], positive regulation of cell killing [GO:0031343], GO:0031643, GO:0032388, GO:0034764, positive regulation of programmed cell death [GO:0043068], GO:0044089, positive regulation of cell differentiation [GO:0045597], positive regulation of cell adhesion [GO:0045785], positive regulation of cell cycle [GO:0045787], positive regulation of establishment of competence for transformation [GO:0045809], positive regulation of cytolysis [GO:0045919], positive regulation of cell activation [GO:0050867], positive regulation of cellular component organization [GO:0051130], positive regulation of sequestering of calcium ion [GO:0051284], positive regulation of cell division [GO:0051781], positive regulation of cell adhesion molecule production [GO:0060355], positive regulation of establishment of bipolar cell polarity [GO:0061173], positive regulation of cellular response to phosphate starvation [GO:0080040], positive regulation of protein targeting to membrane [GO:0090314], positive regulation of vesicle docking [GO:0106022], positive regulation of aggregation involved in sorocarp development [GO:0110013], positive regulation of cellular response to heat [GO:1900036], GO:1900039, positive regulation of cellular response to insulin stimulus [GO:1900078], positive regulation of single-species biofilm formation [GO:1900192], positive regulation of phenotypic switching [GO:1900241], positive regulation of cellular response to oxidative stress [GO:1900409], GO:1902027, positive regulation of response to cell cycle checkpoint signaling [GO:1902146], GO:1902458, positive regulation of synaptic vesicle transport [GO:1902805], positive regulation of horizontal cell localization [GO:1902874], positive regulation of melanosome transport [GO:1902910], positive regulation of actin filament-based movement [GO:1903116], GO:1903334, positive regulation of cell wall organization or biogenesis [GO:1903340], positive regulation of secretion by cell [GO:1903532], GO:1903833, positive regulation of actin filament severing [GO:1903920], positive regulation of transcytosis [GO:1904300], positive regulation of spore germination [GO:1904361], positive regulation of vascular associated smooth muscle cell dedifferentiation [GO:1905176], positive regulation of protein localization to membrane [GO:1905477], positive regulation of cellular response to manganese ion [GO:1905804], positive regulation of cellular response to gamma radiation [GO:1905845], positive regulation of cellular response to oxidopamine [GO:1905848], positive regulation of cellular response to very-low-density lipoprotein particle stimulus [GO:1905889], GO:1905898, positive regulation of cell fate determination [GO:1905935], positive regulation of cellular response to alcohol [GO:1905959], positive regulation of cell motility [GO:2000147], positive regulation of ribonucleoprotein complex localization [GO:2000199], GO:2000522, positive regulation of cellular response to X-ray [GO:2000685], positive regulation of establishment or maintenance of cell polarity regulating cell shape [GO:2000771], positive regulation of cellular senescence [GO:2000774], GO:2001040, GO:2001043 Sources: GOC:jid Definition: Any process that activates or increases the frequency, rate or extent of a cellular process, any of those that are carried out at the cellular level, but are not necessarily restricted to a single cell. For example, cell communication occurs among more than one cell, but occurs at the cellular level. Relationships: is a type of GO:0048518; is a type of regulation of cellular process [GO:0050794]; positively regulates cellular process [GO:0009987] Also known as: positive regulation of cellular physiological process, up regulation of cellular process, up-regulation of cellular process, upregulation of cellular process, activation of cellular process, stimulation of cellular process